{
  "gene_symbol": "FGF13",
  "gene_name": "Fibroblast growth factor 13",
  "term_id": "GO:0017080",
  "gene": "UniProtKB:Q92913",
  "term_label": "sodium channel regulator activity"
}